{
  "gene_symbol": "CPA4",
  "term_id": "GO:0005615",
  "gene_name": "Carboxypeptidase A4",
  "term_label": "extracellular space",
  "gene": "UniProtKB:Q9UI42"
}